{
  "term_label": "coreceptor activity",
  "gene_name": "Tumor necrosis factor receptor superfamily member 16",
  "term_id": "GO:0015026",
  "gene": "UniProtKB:P08138",
  "gene_symbol": "NGFR"
}